{
  "term_id": "GO:0031838",
  "gene_symbol": "HBZ",
  "gene_name": "Hemoglobin subunit zeta",
  "term_label": "haptoglobin-hemoglobin complex",
  "gene": "UniProtKB:P02008"
}